{
  "gene_symbol": "OR13C7",
  "term_label": "plasma membrane",
  "term_id": "GO:0005886",
  "gene_name": "Olfactory receptor 13C7",
  "gene": "UniProtKB:P0DN81"
}